regulation of terminal button organization [GO:2000331] (biological process) Subtypes: negative regulation of terminal button organization [GO:1901613], positive regulation of terminal button organization [GO:1901614] Sources: GOC:BHF, GOC:mah Definition: Any process that modulates the frequency, rate or extent of terminal button organization. Relationships: is a type of regulation of presynapse organization [GO:0099174]; regulates terminal button organization [GO:0072553] Also known as: regulation of bouton organization, regulation of presynaptic bouton organization, regulation of synaptic bouton organization, regulation of terminal bouton organization, regulation of terminal button organisation